{
  "gene_symbol": "GTF2H5",
  "gene": "UniProtKB:Q6ZYL4",
  "gene_name": "General transcription factor IIH subunit 5",
  "term_label": "transcription factor TFIIH core complex",
  "term_id": "GO:0000439"
}